acyl-CoA 6-desaturase activity [GO:0016213] (MF) References: PMID:12713571, PMID:7212717 Sources: EC:1.14.19.3 Definition: Catalysis of the introduction of a cis double bond at carbon 6 of acyl-CoAs, introducing a new double bond between a pre-existing double bond and the carboxyl-end of the fatty acid. Specific reactions include: (9Z,12Z)-octadecadienoyl-CoA + 2 Fe(II)-[cytochrome b5] + 2 H+ + O2 = (6Z,9Z,12Z)-octadecatrienoyl-CoA + 2 Fe(III)-[cytochrome b5] + 2 H2O; and (9Z,12Z,15Z)-octadecatrienoyl-CoA + 2 Fe(II)-[cytochrome b5] + O2 + 2 H+ = (6Z,9Z,12Z,15Z)-octadecatetraenoyl-CoA + 2 Fe(III)-[cytochrome b5] + 2 H2O. Also known as: delta(6)-acyl CoA desaturase activity, delta(6)-desaturase activity, delta(6)-fatty acyl-CoA desaturase activity, fatty acid 6-desaturase activity, fatty acid delta(6)-desaturase activity, long-chain fatty acid delta(6)-desaturase activity, linoleoyl CoA desaturase activity, linoleoyl-CoA desaturase activity, linoleoyl-coenzyme A desaturase activity, delta6-acyl CoA desaturase activity, delta6-desaturase activity, delta6-fatty acyl-CoA desaturase activity, fatty acid delta6-desaturase activity, linoleate desaturase activity, linoleic acid desaturase activity, linoleic desaturase activity, long-chain fatty acid delta6-desaturase activity Relationships: is a type of acyl-CoA desaturase activity [GO:0016215]